{
  "gene_symbol": "MFSD6",
  "gene_name": "Major facilitator superfamily domain-containing protein 6",
  "term_id": "GO:0042590",
  "term_label": "antigen processing and presentation of exogenous peptide antigen via MHC class I",
  "gene": "UniProtKB:Q6ZSS7"
}